{
  "term_id": "GO:0042981",
  "gene_symbol": "USP17L19",
  "gene_name": "Ubiquitin carboxyl-terminal hydrolase 17-like protein 19",
  "gene": "UniProtKB:D6RCP7",
  "term_label": "regulation of apoptotic process"
}